{
  "term_label": "Unknown cellular component",
  "term_id": "UNKNOWN:0003",
  "gene": "UniProtKB:Q9H5V9",
  "gene_name": "STING ER exit protein",
  "gene_symbol": "STEEP1"
}